{
  "gene_name": "Large ribosomal subunit protein bL21m",
  "term_id": "GO:0003735",
  "gene": "UniProtKB:Q7Z2W9",
  "gene_symbol": "MRPL21",
  "term_label": "structural constituent of ribosome"
}